{
  "gene": "UniProtKB:Q15583",
  "gene_name": "Homeobox protein TGIF1",
  "term_id": "GO:0000122",
  "gene_symbol": "TGIF1",
  "term_label": "negative regulation of transcription by RNA polymerase II"
}